{
  "term_label": "DNA-binding transcription factor activity, RNA polymerase II-specific",
  "gene_symbol": "RBAK",
  "gene_name": "RB-associated KRAB zinc finger protein",
  "gene": "UniProtKB:Q9NYW8",
  "term_id": "GO:0000981"
}